{
  "gene": "UniProtKB:O43617",
  "term_id": "GO:0006891",
  "term_label": "intra-Golgi vesicle-mediated transport",
  "gene_name": "Trafficking protein particle complex subunit 3",
  "gene_symbol": "TRAPPC3"
}